{
  "gene_symbol": "SESTD1",
  "gene": "UniProtKB:Q86VW0",
  "term_label": "phosphatidylinositol-4,5-bisphosphate binding",
  "gene_name": "SEC14 domain and spectrin repeat-containing protein 1",
  "term_id": "GO:0005546"
}